{
  "term_label": "endoplasmic reticulum tubular network",
  "gene_symbol": "PARP8",
  "gene_name": "Protein mono-ADP-ribosyltransferase PARP8",
  "gene": "UniProtKB:Q8N3A8",
  "term_id": "GO:0071782"
}